{
  "gene": "UniProtKB:Q96ID5",
  "term_id": "GO:0098839",
  "term_label": "postsynaptic density membrane",
  "gene_symbol": "IGSF21",
  "gene_name": "Immunoglobulin superfamily member 21"
}